{
  "term_label": "intracellular signal transduction",
  "gene": "UniProtKB:Q14449",
  "gene_symbol": "GRB14",
  "term_id": "GO:0035556",
  "gene_name": "Growth factor receptor-bound protein 14"
}